photoreceptor cell development [GO:0042461] (biological process) Relationships: is a type of neuron development [GO:0048666]; is part of photoreceptor cell differentiation [GO:0046530] Subtypes: GO:0042462, ocellus photoreceptor cell development [GO:0042463] Also known as: photoreceptor morphogenesis Sources: GOC:go_curators Definition: Development of a photoreceptor, a cell that responds to incident electromagnetic radiation, particularly visible light.